response to monosaccharide [GO:0034284] (biological process) Also known as: response to monosaccharide stimulus Sources: GOC:mah Definition: Any process that results in a change in state or activity of a cell or an organism (in terms of movement, secretion, enzyme production, gene expression, etc.) as a result of a monosaccharide stimulus. Subtypes: response to hexose [GO:0009746], response to L-ascorbic acid [GO:0033591], detection of monosaccharide stimulus [GO:0034287], cellular response to monosaccharide stimulus [GO:0071326], response to glyceraldehyde [GO:1905630] Relationships: is a type of GO:0009743